mesenchymal to epithelial transition involved in mesonephros morphogenesis [GO:0061261] (BP) Sources: GOC:mtg_kidney_jan10 Definition: A transition where a mesenchymal cell establishes apical/basolateral polarity, forms intercellular adhesive junctions, synthesizes basement membrane components and becomes an epithelial cell that will contribute to the shaping of the mesonephros. Relationships: is a type of epithelial cell differentiation involved in kidney development [GO:0035850]; is a type of mesenchymal to epithelial transition [GO:0060231]; is a type of GO:0061208; BFO_0000050 GO:0061206 Subtypes: mesenchymal to epithelial transition involved in mesonephric renal vesicle formation [GO:0061271] Also known as: mesonephric mesenchyme to epithelial transition Regulation: RO_0002211 by regulation of mesenchymal to epithelial transition involved in mesonephros morphogenesis [GO:2000084]; negatively regulated by negative regulation of mesenchymal to epithelial transition involved in mesonephros morphogenesis [GO:2000085]; positively regulated by GO:2000086